positive regulation of L-threonine import across plasma membrane [GO:1900928] (biological process) Sources: GOC:TermGenie Relationships: is a type of positive regulation of organic acid transport [GO:0032892]; is a type of GO:0034764; is a type of positive regulation of amino acid transport [GO:0051957]; is a type of regulation of L-threonine import across plasma membrane [GO:1900926]; positively regulates L-threonine import across plasma membrane [GO:1903807] Definition: Any process that activates or increases the frequency, rate or extent of L-threonine import into cell. Also known as: positive regulation of L-threonine import, up regulation of L-threonine import, up-regulation of L-threonine import, upregulation of L-threonine import, activation of L-threonine import, activation of L-threonine uptake, positive regulation of L-threonine uptake, up regulation of L-threonine uptake, up-regulation of L-threonine uptake, upregulation of L-threonine uptake